asparaginyl-tRNA aminoacylation [GO:0006421] (biological process) Relationships: is a type of tRNA aminoacylation for protein translation [GO:0006418] Subtypes: mitochondrial asparaginyl-tRNA aminoacylation [GO:0070145] Sources: GOC:mcc, ISBN:0716730510 Definition: The process of coupling asparagine to asparaginyl-tRNA, catalyzed by asparaginyl-tRNA synthetase. The asparaginyl-tRNA synthetase is a class-II synthetase. The activated amino acid is transferred to the 3'-OH group of an asparagine-accetping tRNA.